response to sorbitol [GO:0072708] (biological process) Relationships: is a type of response to carbohydrate [GO:0009743] Definition: Any process that results in a change in state or activity of a cell or an organism (in terms of movement, secretion, enzyme production, gene expression, etc.) as a result of a sorbitol stimulus. Sources: GOC:mah Subtypes: GO:0072709 Also known as: response to glucitol